{
  "gene_symbol": "PGD",
  "term_id": "GO:0004616",
  "term_label": "phosphogluconate dehydrogenase (decarboxylating) activity",
  "gene_name": "6-phosphogluconate dehydrogenase, decarboxylating",
  "gene": "UniProtKB:P52209"
}